{
  "gene_symbol": "SNIP1",
  "gene": "UniProtKB:Q8TAD8",
  "term_label": "nucleus",
  "term_id": "GO:0005634",
  "gene_name": "Smad nuclear-interacting protein 1"
}